tRNA ligase activator activity [GO:0140733] (molecular function) References: PMID:30943413 Relationships: is a type of enzyme activator activity [GO:0008047]; is a type of ligase regulator activity [GO:0055103]; RO_0002213 GO:0004812 Definition: Binds to and increases the activity of a tRNA ligase.